{
  "gene_symbol": "ADAMTSL1",
  "gene": "UniProtKB:Q8N6G6",
  "term_id": "UNKNOWN:0003",
  "term_label": "Unknown cellular component",
  "gene_name": "ADAMTS-like protein 1"
}